leucophore differentiation [GO:0048772] (biological process) Relationships: is a type of pigment cell differentiation [GO:0050931] Definition: The process in which a relatively unspecialized cell acquires the specialized features of a leucophore cell. Leucophores are pigment cells derived from the neural crest. They contain uric acid or other purine crystals, deposited in stacks called leucosomes. This gives them a white appearance. Regulation: regulated by regulation of leucophore differentiation [GO:0048775]; RO_0002212 by negative regulation of leucophore differentiation [GO:0048776]; positively regulated by positive regulation of leucophore differentiation [GO:0048777] Sources: GOC:jid, GOC:mh Also known as: leucophore cell differentiation